{
  "term_label": "structural constituent of chromatin",
  "gene_symbol": "LMNTD2",
  "term_id": "GO:0030527",
  "gene_name": "Lamin tail domain-containing protein 2",
  "gene": "UniProtKB:Q8IXW0"
}